regulation of natural killer cell mediated immune response to tumor cell [GO:0002855] (biological process) Subtypes: negative regulation of natural killer cell mediated immune response to tumor cell [GO:0002856], GO:0002857, regulation of natural killer cell mediated cytotoxicity directed against tumor cell target [GO:0002858] Sources: GOC:add Relationships: is a type of regulation of natural killer cell mediated immunity [GO:0002715]; is a type of regulation of immune response to tumor cell [GO:0002837]; regulates natural killer cell mediated immune response to tumor cell [GO:0002423] Definition: Any process that modulates the frequency, rate, or extent of natural killer cell mediated immune response to a tumor cell.